fructose:proton symporter activity [GO:0055054] (molecular function) Sources: GOC:ct Relationships: is a type of GO:0005353; is a type of GO:0009679 Definition: Enables the transfer of a solute or solutes from one side of a membrane to the other according to the reaction: fructose + H+ = fructose + H+. Also known as: fructose:hydrogen symporter activity